{
  "gene": "UniProtKB:Q96P67",
  "term_id": "UNKNOWN:0002",
  "term_label": "Unknown biological process",
  "gene_symbol": "GPR82",
  "gene_name": "Probable G-protein coupled receptor 82"
}